{
  "gene_symbol": "ALKAL2",
  "gene": "UniProtKB:Q6UX46",
  "term_label": "receptor signaling protein tyrosine kinase activator activity",
  "term_id": "GO:0030298",
  "gene_name": "ALK and LTK ligand 2"
}